{
  "term_id": "UNKNOWN:0002",
  "term_label": "Unknown biological process",
  "gene_symbol": "LINC00615",
  "gene": "UniProtKB:Q96LM1",
  "gene_name": "Putative uncharacterized protein encoded by LINC00615"
}